{
  "gene_symbol": "EFCAB2",
  "gene": "UniProtKB:Q5VUJ9",
  "term_id": "UNKNOWN:0002",
  "term_label": "Unknown biological process",
  "gene_name": "Dynein regulatory complex protein 8"
}